positive regulation of PERK-mediated unfolded protein response [GO:1903899] (biological process) Definition: Any process that activates or increases the frequency, rate or extent of the PERK-mediated unfolded protein response. Also known as: positive regulation of PERK branch of UPR, positive regulation of PKR-like ER kinase signal transduction, positive regulation of UPR signaling by PERK stress sensor, positive regulation of endoplasmic reticulum unfolded protein response; PERK signaling, up regulation of PERK branch of UPR, up regulation of PERK-mediated unfolded protein response, up regulation of PKR-like ER kinase signal transduction, up regulation of UPR signaling by PERK stress sensor, up regulation of endoplasmic reticulum unfolded protein response; PERK signaling, up-regulation of PERK branch of UPR, up-regulation of PERK-mediated unfolded protein response, up-regulation of PKR-like ER kinase signal transduction, up-regulation of UPR signaling by PERK stress sensor, up-regulation of endoplasmic reticulum unfolded protein response; PERK signaling, upregulation of PERK branch of UPR, upregulation of PERK-mediated unfolded protein response, upregulation of PKR-like ER kinase signal transduction, upregulation of UPR signaling by PERK stress sensor, upregulation of endoplasmic reticulum unfolded protein response; PERK signaling, activation of PERK branch of UPR, activation of PERK-mediated unfolded protein response, activation of PKR-like ER kinase signal transduction, activation of UPR signaling by PERK stress sensor, activation of endoplasmic reticulum unfolded protein response; PERK signaling, activation of PERK signaling in response to endoplasmic reticulum stress, positive regulation of EIF2AK3-mediated unfolded protein response, positive regulation of PERK signaling in response to endoplasmic reticulum stress, up regulation of PERK signaling in response to endoplasmic reticulum stress, up-regulation of PERK signaling in response to endoplasmic reticulum stress, upregulation of PERK signaling in response to endoplasmic reticulum stress References: PMID:22013210 Sources: GOC:PARL, GOC:TermGenie, GOC:bf, GO_REF:0000058 Relationships: is a type of positive regulation of endoplasmic reticulum unfolded protein response [GO:1900103]; is_a regulation of PERK-mediated unfolded protein response [GO:1903897]; positively regulates PERK-mediated unfolded protein response [GO:0036499]